{
  "term_label": "Unknown molecular function",
  "gene": "UniProtKB:Q9HBL7",
  "term_id": "UNKNOWN:0001",
  "gene_name": "Plasminogen receptor (KT)",
  "gene_symbol": "PLGRKT"
}